forebrain dorsal/ventral pattern formation [GO:0021798] (biological process) Sources: GOC:cls, GOC:dgh, GOC:dph, GOC:jid, GO_REF:0000021 Definition: The formation of specific regional progenitor domains along the dorsal-ventral axis in the developing forebrain. Relationships: is a type of dorsal/ventral pattern formation [GO:0009953]; is part of forebrain regionalization [GO:0021871] Also known as: forebrain dorsal-ventral pattern formation, forebrain dorsoventral pattern formation